{
  "gene_symbol": "MTHFD1",
  "term_label": "methylenetetrahydrofolate dehydrogenase (NADP+) activity",
  "term_id": "GO:0004488",
  "gene": "UniProtKB:P11586",
  "gene_name": "C-1-tetrahydrofolate synthase, cytoplasmic"
}